{
  "gene_name": "Phospholipase A2",
  "term_id": "GO:0005102",
  "gene_symbol": "PLA2G1B",
  "gene": "UniProtKB:P04054",
  "term_label": "signaling receptor binding"
}